{
  "gene_symbol": "ALG3",
  "gene": "UniProtKB:Q92685",
  "term_label": "dol-P-Man:Man(5)GlcNAc(2)-PP-Dol alpha-1,3-mannosyltransferase activity",
  "gene_name": "Dol-P-Man:Man(5)GlcNAc(2)-PP-Dol alpha-1,3-mannosyltransferase",
  "term_id": "GO:0052925"
}